{
  "gene": "UniProtKB:Q8WYK0",
  "gene_symbol": "ACOT12",
  "gene_name": "Acetyl-coenzyme A thioesterase",
  "term_id": "GO:0003986",
  "term_label": "acetyl-CoA hydrolase activity"
}